spindle pole body [GO:0005816] (cellular component) Subtypes: meiotic spindle pole body [GO:0035974], GO:0044732 Definition: The microtubule organizing center in fungi; functionally homologous to the animal cell centrosome. Also known as: SPB Relationships: is_a microtubule organizing center [GO:0005815] Sources: ISBN:0879693568